{
  "term_label": "hormone activity",
  "term_id": "GO:0005179",
  "gene_name": "Leptin",
  "gene": "UniProtKB:P41159",
  "gene_symbol": "LEP"
}